{
  "term_label": "Unknown biological process",
  "gene_symbol": "Q3C1V9",
  "gene": "UniProtKB:Q3C1V9",
  "term_id": "UNKNOWN:0002",
  "gene_name": "Putative uncharacterized protein ENSP00000334305"
}